{
  "gene": "UniProtKB:P26992",
  "gene_symbol": "CNTFR",
  "term_id": "GO:0097059",
  "gene_name": "Ciliary neurotrophic factor receptor subunit alpha",
  "term_label": "CNTFR-CLCF1 complex"
}